{
  "gene_symbol": "COMT",
  "gene_name": "Catechol O-methyltransferase",
  "gene": "UniProtKB:P21964",
  "term_id": "GO:0030425",
  "term_label": "dendrite"
}